{
  "term_label": "plasma membrane",
  "gene_name": "Synaptotagmin-3",
  "gene": "UniProtKB:Q9BQG1",
  "gene_symbol": "SYT3",
  "term_id": "GO:0005886"
}